establishment of plant organ orientation [GO:0090707] (biological process) Relationships: is a type of GO:0048560; is part of plant organ morphogenesis [GO:1905392] Subtypes: GO:0048559 Sources: GOC:tb Definition: The process that determines the orientation of a plant organ or tissue with reference to an axis.